{
  "term_id": "GO:0016477",
  "term_label": "cell migration",
  "gene_symbol": "CLEC14A",
  "gene": "UniProtKB:Q86T13",
  "gene_name": "C-type lectin domain family 14 member A"
}